transcription coregulator activity [GO:0003712] (molecular function) Subtypes: transcription coactivator activity [GO:0003713], GO:0003714 Also known as: transcription cofactor activity, transcription coreceptor activity, transcriptional co-regulator, nuclear receptor coreceptor activity, RNA polymerase II transcriptional cofactor activity References: PMID:10213677, PMID:16858867, PMID:24203923, PMID:25957681 Sources: GOC:txnOH-2018, Wikipedia:Transcription_coregulator Relationships: is_a protein-macromolecule adaptor activity [GO:0030674]; is a type of transcription regulator activity [GO:0140110] Definition: A transcription regulator activity that modulates the transcription of specific gene sets via binding to a DNA-binding transcription factor at a specific genomic locus, either on its own or as part of a complex. Coregulators often act by altering chromatin structure and modifications. For example, one class of transcription coregulators modifies chromatin structure through covalent modification of histones. A second class remodels the conformation of chromatin in an ATP-dependent fashion. A third class modulates interactions of DNA-bound DNA-binding transcription factors with other transcription coregulators. Note: Usage guidance: Most transcription coregulators do not bind DNA. Those that do usually bind DNA either in a non-specific or non-direct manner. If a protein binds DNA specifically, consider annotating to GO:0003700 DNA binding transcription factor activity.